growth cone filopodium [GO:1990812] (cellular component) Definition: A thin, stiff protrusion extended by the leading edge of an axonal or dendritic growth cone. References: PMID:25598228 Relationships: is a type of GO:0030175; is a type of neuron projection [GO:0043005]; is part of growth cone [GO:0030426]